{
  "term_label": "cytokine receptor activity",
  "term_id": "GO:0004896",
  "gene_name": "Interleukin-12 receptor subunit beta-1",
  "gene": "UniProtKB:P42701",
  "gene_symbol": "IL12RB1"
}